L-ornithine transmembrane transport [GO:1903352] (biological process) Definition: The directed movement of L-ornithine across a membrane. References: PMID:8195186 Sources: GOC:TermGenie, GOC:krc, GO_REF:0000069 Relationships: is a type of ornithine transport [GO:0015822]; is_a L-alpha-amino acid transmembrane transport [GO:1902475] Subtypes: L-ornithine transmembrane export from vacuole [GO:0089706], L-ornithine import across plasma membrane [GO:0097640], mitochondrial L-ornithine transmembrane transport [GO:1990575]